{
  "gene_symbol": "PRL",
  "term_id": "GO:0005615",
  "gene_name": "Prolactin",
  "gene": "UniProtKB:P01236",
  "term_label": "extracellular space"
}